positive regulation of conidiophore development [GO:0070795] (BP) Definition: Any process that activates or increases the frequency, rate or extent of conidiophore development, a process that leads to the formation of a conidiophore. The conidiophore is a specialized hypha that extends aerially from the growth substrate and bears conidia, or asexual spores. Subtypes: GO:0070801 Relationships: is a type of regulation of conidiophore development [GO:0070793]; is a type of GO:0075261; RO_0002213 GO:0070787 Sources: GOC:mah